{
  "gene": "UniProtKB:Q93091",
  "term_label": "defense response to Gram-negative bacterium",
  "gene_name": "Ribonuclease K6",
  "term_id": "GO:0050829",
  "gene_symbol": "RNASE6"
}